wishful thinking binding [GO:0005117] (MF) Definition: Binding to wishful thinking (Wit), a type II bone morphogenic protein receptor. References: PMID:11856529 Sources: GOC:ceb Also known as: Wit binding, SE20 receptor binding, Wit ligand, wishful thinking ligand Relationships: is a type of GO:0005102